{
  "term_label": "cytosol",
  "term_id": "GO:0005829",
  "gene_name": "Cytosolic phospholipase A2 delta",
  "gene": "UniProtKB:Q86XP0",
  "gene_symbol": "PLA2G4D"
}